{
  "gene": "UniProtKB:Q9H607",
  "term_id": "UNKNOWN:0001",
  "gene_symbol": "OCEL1",
  "gene_name": "Occludin_ELL domain-containing protein 1",
  "term_label": "Unknown molecular function"
}